interleukin-4 receptor binding [GO:0005136] (molecular function) Also known as: IL-4, interleukin-4 receptor ligand Relationships: is a type of cytokine receptor binding [GO:0005126]; is a type of growth factor receptor binding [GO:0070851] Sources: GOC:ai Definition: Binding to an interleukin-4 receptor.